response to gold(3+) [GO:1904311] (biological process) Definition: Any process that results in a change in state or activity of a cell or an organism (in terms of movement, secretion, enzyme production, gene expression, etc.) as a result of a gold(3+) stimulus. References: PMID:16206274 Sources: GOC:TermGenie, GO_REF:0000071 Relationships: is a type of response to metal ion [GO:0010038] Subtypes: cellular response to gold(3+) [GO:1904312]